{
  "gene_symbol": "PYY",
  "term_label": "extracellular space",
  "gene": "UniProtKB:P10082",
  "term_id": "GO:0005615",
  "gene_name": "Peptide YY"
}